regulation of rhamnose catabolic process [GO:0043463] (biological process) Definition: Any process that modulates the frequency, rate or extent of the chemical reactions and pathways resulting in the breakdown of rhamnose, the hexose 6-deoxy-L-mannose. Sources: GOC:jl Also known as: regulation of rhamnose breakdown, regulation of rhamnose catabolism, regulation of rhamnose degradation Relationships: is a type of GO:0043470; is a type of GO:0062012; regulates rhamnose catabolic process [GO:0019301]